nascent polypeptide-associated complex [GO:0005854] (cellular component) Definition: A heterodimeric protein complex that can reversibly bind to ribosomes, and is located in direct proximity to newly synthesized polypeptide chains as they emerge from the ribosome. Relationships: is a type of protein-containing complex [GO:0032991]; is part of cytoplasm [GO:0005737] References: PMID:12475173, PMID:7568149 Also known as: NAC, NACA